{
  "term_id": "UNKNOWN:0002",
  "gene_name": "Uncharacterized protein CD300LD-AS1",
  "gene": "UniProtKB:Q96MU5",
  "term_label": "Unknown biological process",
  "gene_symbol": "CD300LD-AS1"
}